{
  "gene_name": "Paralemmin-1",
  "term_id": "UNKNOWN:0001",
  "gene_symbol": "PALM",
  "term_label": "Unknown molecular function",
  "gene": "UniProtKB:O75781"
}